{
  "gene_name": "Olfactory receptor 7D4",
  "gene": "UniProtKB:Q8NG98",
  "term_label": "plasma membrane",
  "gene_symbol": "OR7D4",
  "term_id": "GO:0005886"
}